{
  "term_id": "GO:0005737",
  "gene_name": "Twinfilin-1",
  "gene_symbol": "TWF1",
  "gene": "UniProtKB:Q12792",
  "term_label": "cytoplasm"
}